{
  "gene_symbol": "PABPC5",
  "gene_name": "Polyadenylate-binding protein 5",
  "term_id": "GO:0005634",
  "term_label": "nucleus",
  "gene": "UniProtKB:Q96DU9"
}